intracellular lipid transport [GO:0032365] (biological process) Definition: The directed movement of lipids within cells. Regulation: RO_0002211 by regulation of intracellular lipid transport [GO:0032377]; negatively regulated by negative regulation of intracellular lipid transport [GO:0032378]; positively regulated by GO:0032379 Relationships: is a type of lipid transport [GO:0006869]; is a type of intracellular transport [GO:0046907] Sources: GOC:mah Subtypes: carnitine shuttle [GO:0006853], long-chain fatty acid import into peroxisome [GO:0015910], intracellular sterol transport [GO:0032366], ER to Golgi ceramide transport [GO:0035621], isopentenyl pyrophosphate import into mitochondrion [GO:0170046], ER to chloroplast lipid transport [GO:1990052]